{
  "gene_symbol": "EIF2AK2",
  "term_label": "cytoplasm",
  "gene_name": "Interferon-induced, double-stranded RNA-activated protein kinase",
  "gene": "UniProtKB:P19525",
  "term_id": "GO:0005737"
}